phosphonoacetaldehyde hydrolase activity [GO:0050194] (molecular function) Relationships: is a type of hydrolase activity, acting on acid carbon-phosphorus bonds [GO:0016827] Also known as: 2-oxoethylphosphonate phosphonohydrolase activity, 2-phosphonoacetylaldehyde phosphonohydrolase activity, phosphonatase activity, phosphonoacetylaldehyde phosphonohydrolase activity Definition: Catalysis of the reaction: H2O + phosphonoacetaldehyde = acetaldehyde + H+ + phosphate. Sources: RHEA:18905